{
  "term_id": "GO:0005886",
  "term_label": "plasma membrane",
  "gene_name": "Kremen protein 1",
  "gene": "UniProtKB:Q96MU8",
  "gene_symbol": "KREMEN1"
}